2-hydroxychromene-2-carboxylate isomerase activity [GO:0018845] (molecular function) Relationships: is_a intramolecular oxidoreductase activity [GO:0016860] Definition: Catalysis of the reaction: 2-hydroxychromene-2-carboxylate = (3E)-4-(2-hydroxyphenyl)-2-oxobut-3-enoate. (3E)-4-(2-hydroxyphenyl)-2-oxobut-3-enoate is also known as trans-o-hydroxybenzylidenepyruvate. Sources: RHEA:27401